superior colliculus development [GO:0061380] (biological process) Relationships: is a type of anatomical structure development [GO:0048856]; is part of corpora quadrigemina development [GO:0061378] Definition: The process whose specific outcome is the progression of the superior colliculus over time, from its formation to the mature structure. The superior colliculus is also known as the optic tectum or simply tectum and is a paired structure that forms a major component of the vertebrate midbrain. Sources: GOC:dph, GOC:yaf